{
  "term_label": "mRNA binding",
  "term_id": "GO:0003729",
  "gene": "UniProtKB:O00267",
  "gene_name": "Transcription elongation factor SPT5",
  "gene_symbol": "SUPT5H"
}